{
  "term_label": "dTDP-glucose 4,6-dehydratase activity",
  "gene_name": "dTDP-D-glucose 4,6-dehydratase",
  "gene_symbol": "TGDS",
  "term_id": "GO:0008460",
  "gene": "UniProtKB:O95455"
}